CMP-N-acetylneuraminate biosynthetic process [GO:0006055] (BP) Definition: The chemical reactions and pathways resulting in the formation of CMP-N-acetylneuraminate, a substance composed of 5-(acetylamino)-3,5-dideoxy-D-glycero-D-galacto-non-3-ulosonic acid in glycosidic linkage with cytidine monophosphate. Sources: GOC:ai Also known as: CMP-N-acetylneuraminate anabolism, CMP-N-acetylneuraminate biosynthesis, CMP-N-acetylneuraminate formation, CMP-N-acetylneuraminate synthesis Relationships: is a type of nucleotide-sugar biosynthetic process [GO:0009226]; is a type of GO:0046381